bacterial cellulose biosynthetic process [GO:0090540] (biological process) Definition: The chemical reactions and pathways resulting in the formation of cellulose, a linear beta1-4 glucan of molecular mass 50-400 kDa with the pyranose units in the -4C1 conformation, as it occurs in certain types of bacteria, mainly Acetobacter, Sarcina ventriculi and Agrobacteria. References: PMID:24097954 Sources: GOC:yaf Also known as: bacterial cellulose biosynthesis Relationships: is a type of cellulose biosynthetic process [GO:0030244]